{
  "gene_symbol": "STEAP2",
  "gene": "UniProtKB:Q8NFT2",
  "term_label": "endosome",
  "term_id": "GO:0005768",
  "gene_name": "Metalloreductase STEAP2"
}